uridine biosynthetic process [GO:0046109] (biological process) Relationships: is a type of GO:0046108; is a type of pyrimidine ribonucleoside biosynthetic process [GO:0046132] Sources: GOC:go_curators Also known as: uridine anabolism, uridine biosynthesis, uridine formation, uridine synthesis Definition: The chemical reactions and pathways resulting in the formation of uridine, uracil riboside, a ribonucleoside very widely distributed but occurring almost entirely as phosphoric esters in ribonucleotides and ribonucleic acids.